{
  "term_id": "GO:0060337",
  "gene": "UniProtKB:Q01628",
  "gene_symbol": "IFITM3",
  "term_label": "type I interferon-mediated signaling pathway",
  "gene_name": "Interferon-induced transmembrane protein 3"
}